{
  "gene_name": "ATP-dependent DNA helicase PIF1",
  "term_id": "UNKNOWN:0003",
  "gene": "UniProtKB:Q9H611",
  "term_label": "Unknown cellular component",
  "gene_symbol": "PIF1"
}